{
  "gene": "UniProtKB:Q8IYV9",
  "gene_symbol": "IZUMO1",
  "term_label": "binding of sperm to zona pellucida",
  "gene_name": "Izumo sperm-egg fusion protein 1",
  "term_id": "GO:0007339"
}